{
  "gene_symbol": "STX5",
  "term_id": "GO:0031201",
  "gene": "UniProtKB:Q13190",
  "term_label": "SNARE complex",
  "gene_name": "Syntaxin-5"
}